{
  "term_id": "GO:0016567",
  "gene_symbol": "CUL4B",
  "gene": "UniProtKB:Q13620",
  "term_label": "protein ubiquitination",
  "gene_name": "Cullin-4B"
}